negative regulation of erythrocyte differentiation [GO:0045647] (biological process) Definition: Any process that stops, prevents, or reduces the frequency, rate or extent of erythrocyte differentiation. Sources: GOC:go_curators Relationships: is a type of negative regulation of myeloid cell differentiation [GO:0045638]; is_a regulation of erythrocyte differentiation [GO:0045646]; negatively regulates erythrocyte differentiation [GO:0030218] Also known as: down regulation of erythrocyte differentiation, down-regulation of erythrocyte differentiation, downregulation of erythrocyte differentiation, negative regulation of RBC differentiation, negative regulation of red blood cell differentiation, inhibition of erythrocyte differentiation